{
  "gene_name": "Glycogen phosphorylase, muscle form",
  "gene": "UniProtKB:P11217",
  "term_label": "cytoplasm",
  "gene_symbol": "PYGM",
  "term_id": "GO:0005737"
}